positive regulation of neurotransmitter uptake [GO:0051582] (BP) Sources: GOC:ai Definition: Any process that activates or increases the frequency, rate or extent of the directed movement of a neurotransmitter into a neuron or glial cell. Also known as: positive regulation of neurotransmitter import, up regulation of neurotransmitter uptake, up-regulation of neurotransmitter uptake, upregulation of neurotransmitter uptake, activation of neurotransmitter uptake, stimulation of neurotransmitter uptake Relationships: is a type of regulation of neurotransmitter uptake [GO:0051580]; is a type of GO:0051590; positively regulates neurotransmitter uptake [GO:0001504] Subtypes: GO:0051613, GO:0051618, positive regulation of amino acid uptake involved in synaptic transmission [GO:0051943], positive regulation of catecholamine uptake involved in synaptic transmission [GO:0051944]